{
  "gene": "UniProtKB:Q2TB90",
  "gene_symbol": "HKDC1",
  "term_id": "GO:0005829",
  "term_label": "cytosol",
  "gene_name": "Hexokinase HKDC1"
}